histone H1 asparagine deamidase activity [GO:0160261] (molecular function) References: PMID:40240600 Definition: Catalysis of the reaction: histone H1 L-asparagine + H2O = histone H1 L-aspartate + NH4+. Relationships: is a type of GO:0160260 Subtypes: histone H1N76/N77 asparagine deamidase activity [GO:0160264]